{
  "gene": "UniProtKB:P51861",
  "term_id": "UNKNOWN:0003",
  "term_label": "Unknown cellular component",
  "gene_name": "Cerebellar degeneration-related antigen 1",
  "gene_symbol": "CDR1"
}